negative regulation of transmembrane receptor protein serine/threonine kinase signaling pathway [GO:0090101] (biological process) Relationships: is a type of negative regulation of signal transduction [GO:0009968]; is a type of regulation of transmembrane receptor protein serine/threonine kinase signaling pathway [GO:0090092]; negatively regulates cell surface receptor protein serine/threonine kinase signaling pathway [GO:0007178] Sources: GOC:dph, GOC:tb Subtypes: negative regulation of transforming growth factor beta receptor signaling pathway [GO:0030512], negative regulation of BMP signaling pathway [GO:0030514], GO:0032926, negative regulation of SMAD protein signal transduction [GO:0060392], GO:1902613 Also known as: negative regulation of transmembrane receptor protein serine/threonine kinase signalling pathway Definition: Any process that decreases the rate, frequency, or extent of the series of molecular signals generated as a consequence of a transmembrane receptor serine/threonine kinase binding to its physiological ligand.